cellular response to bisphenol A [GO:1903926] (biological process) Definition: Any process that results in a change in state or activity of a cell (in terms of movement, secretion, enzyme production, gene expression, etc.) as a result of a bisphenol A stimulus. Relationships: is a type of cellular response to oxygen-containing compound [GO:1901701]; is a type of response to bisphenol A [GO:1903925] References: PMID:22957036 Sources: GOC:TermGenie, GO_REF:0000071